fructose export from vacuole to cytoplasm [GO:1902334] (biological process) Also known as: fructose transport from vacuole to cytoplasm References: PMID:23583552 Sources: GOC:TermGenie Definition: The directed movement of fructose from vacuole to cytoplasm. Relationships: is a type of fructose transmembrane transport [GO:0015755]; is a type of vacuolar transmembrane transport [GO:0034486]